{
  "term_id": "GO:0030042",
  "term_label": "actin filament depolymerization",
  "gene_symbol": "MICAL2",
  "gene": "UniProtKB:O94851",
  "gene_name": "[F-actin]-monooxygenase MICAL2"
}